primary cell wall cellulose synthase complex [GO:0044567] (cellular component) Definition: A large, multimeric protein complex which catalyzes the biosynthesis of cellulose for the plant primary cell wall. In Arabidopsis, contains the essential component proteins CESA1 and -3, and a CESA6-related protein. Also known as: primary cell wall CESA complex, primary cell-wall cellulose synthase complex Relationships: is a type of cellulose synthase complex [GO:0010330] References: PMID:17878302, PMID:21307367 Sources: GOC:mengo_curators, GOC:tt